{
  "term_label": "Unknown biological process",
  "gene_symbol": "SPDYE2B",
  "term_id": "UNKNOWN:0002",
  "gene_name": "Speedy protein E2B",
  "gene": "UniProtKB:A6NHP3"
}